prosthetic group catabolic process [GO:0051190] (biological process) Definition: The chemical reactions and pathways resulting in the breakdown of a prosthetic group, the non-amino acid portion of certain protein molecules. Prosthetic groups may be inorganic or organic and are usually required for the biological activity of the protein. Sources: GOC:ai Also known as: coenzyme and prosthetic group catabolic process, coenzyme and prosthetic group catabolism, prosthetic group breakdown, prosthetic group catabolism, prosthetic group degradation Relationships: is a type of GO:0009056; is a type of prosthetic group metabolic process [GO:0051189]; is part of protein catabolic process [GO:0030163]